{
  "gene_symbol": "OR7G2",
  "term_id": "GO:0007165",
  "term_label": "signal transduction",
  "gene_name": "Olfactory receptor 7G2",
  "gene": "UniProtKB:Q8NG99"
}